{
  "gene_symbol": "SAG",
  "term_label": "G protein-coupled receptor binding",
  "term_id": "GO:0001664",
  "gene": "UniProtKB:P10523",
  "gene_name": "S-arrestin"
}